{
  "gene": "UniProtKB:Q9UL63",
  "term_label": "cytoplasm",
  "gene_name": "Muskelin",
  "term_id": "GO:0005737",
  "gene_symbol": "MKLN1"
}